{
  "term_label": "kinetochore",
  "term_id": "GO:0000776",
  "gene": "UniProtKB:Q9NXR1",
  "gene_symbol": "NDE1",
  "gene_name": "Nuclear distribution protein nudE homolog 1"
}